xenobiotic detoxification by transmembrane export across the cell outer membrane [GO:0140330] (biological process) Definition: A process that reduces or removes the toxicity of a xenobiotic by exporting it outside the cell through the outer membrane. References: PMID:11948170 Relationships: is a type of xenobiotic transport [GO:0042908]; is a type of GO:0140317; is part of detoxification [GO:0098754]